{
  "term_label": "Unknown molecular function",
  "gene_symbol": "NXT2",
  "term_id": "UNKNOWN:0001",
  "gene": "UniProtKB:Q9NPJ8",
  "gene_name": "NTF2-related export protein 2"
}